{
  "gene_name": "Signal transducer and activator of transcription 1-alpha_beta",
  "gene_symbol": "STAT1",
  "term_label": "cytoplasm",
  "term_id": "GO:0005737",
  "gene": "UniProtKB:P42224"
}